{
  "term_id": "GO:0034982",
  "gene_name": "Paraplegin",
  "gene_symbol": "SPG7",
  "gene": "UniProtKB:Q9UQ90",
  "term_label": "mitochondrial protein processing"
}